{
  "gene": "UniProtKB:Q9HAQ2",
  "gene_name": "Kinesin-like protein KIF9",
  "term_label": "microtubule motor activity",
  "term_id": "GO:0003777",
  "gene_symbol": "KIF9"
}